{
  "gene": "UniProtKB:P06727",
  "term_id": "GO:0042627",
  "term_label": "chylomicron",
  "gene_name": "Apolipoprotein A-IV",
  "gene_symbol": "APOA4"
}